{
  "gene_symbol": "EYA1",
  "gene_name": "Eyes absent homolog 1",
  "term_label": "protein tyrosine phosphatase activity",
  "term_id": "GO:0004725",
  "gene": "UniProtKB:Q99502"
}